{
  "term_label": "plasma membrane",
  "gene_name": "Monocarboxylate transporter 10",
  "gene": "UniProtKB:Q8TF71",
  "gene_symbol": "SLC16A10",
  "term_id": "GO:0005886"
}